{
  "gene_symbol": "PSMA7",
  "term_label": "nucleus",
  "gene": "UniProtKB:O14818",
  "term_id": "GO:0005634",
  "gene_name": "Proteasome subunit alpha type-7"
}